{
  "term_label": "osteoclast differentiation",
  "gene_symbol": "OSTM1",
  "gene": "UniProtKB:Q86WC4",
  "gene_name": "Osteopetrosis-associated transmembrane protein 1",
  "term_id": "GO:0030316"
}